{
  "gene_symbol": "TNPO2",
  "gene": "UniProtKB:O14787",
  "gene_name": "Transportin-2",
  "term_id": "GO:0005634",
  "term_label": "nucleus"
}